monomeric IgA immunoglobulin complex [GO:0071748] (cellular component) Note: Note that an IgA immunoglobulin complex has the function of antigen binding if a suitable antigen is available. Definition: A protein complex composed of two identical immunoglobulin heavy chains of an IgA isotype and two identical immunoglobulin light chains, held together by disulfide bonds, and present in the extracellular space, in mucosal areas or other tissues, or circulating in the blood or lymph. Also known as: monomeric IgA antibody, monomeric IgA1 antibody, monomeric IgA2 antibody References: PMID:16362985 Sources: GOC:add, ISBN:0781765196 Relationships: is a type of IgA immunoglobulin complex, circulating [GO:0071746]